positive regulation of very-low-density lipoprotein particle clearance [GO:0110119] (biological process) Relationships: is a type of regulation of very-low-density lipoprotein particle clearance [GO:0010915]; is a type of positive regulation of lipoprotein particle clearance [GO:0010986]; RO_0002213 GO:0034447 References: PMID:25510864 Sources: GOC:BHF, GOC:BHF_miRNA, GOC:rph Definition: Any process that increases the frequency, rate or extent of very-low-density lipoprotein particle clearance.